{
  "gene": "UniProtKB:Q92615",
  "gene_name": "La-related protein 4B",
  "term_label": "cytoplasmic stress granule",
  "term_id": "GO:0010494",
  "gene_symbol": "LARP4B"
}